{
  "gene": "UniProtKB:Q4FZB7",
  "gene_name": "Histone-lysine N-methyltransferase KMT5B",
  "term_label": "histone H4K20 methyltransferase activity",
  "gene_symbol": "KMT5B",
  "term_id": "GO:0042799"
}